{
  "term_id": "GO:0005886",
  "term_label": "plasma membrane",
  "gene_name": "Angiomotin-like protein 1",
  "gene_symbol": "AMOTL1",
  "gene": "UniProtKB:Q8IY63"
}